neuronal dense core vesicle organization [GO:0099014] (biological process) Sources: GOC:dos Relationships: is a type of dense core granule organization [GO:0061109] Definition: A process that is carried out at the cellular level which results in the assembly, arrangement of constituent parts, or disassembly of a neuronal dense core vesicle.